{
  "gene": "UniProtKB:O43432",
  "gene_name": "Eukaryotic translation initiation factor 4 gamma 3",
  "term_id": "GO:0006413",
  "gene_symbol": "EIF4G3",
  "term_label": "translational initiation"
}